{
  "gene": "UniProtKB:H3BV60",
  "gene_name": "Transforming growth factor-beta receptor type 3-like protein",
  "gene_symbol": "TGFBR3L",
  "term_id": "GO:0001837",
  "term_label": "epithelial to mesenchymal transition"
}